{
  "gene": "UniProtKB:Q9NPJ4",
  "term_id": "UNKNOWN:0001",
  "term_label": "Unknown molecular function",
  "gene_name": "Proline-rich nuclear receptor coactivator 2",
  "gene_symbol": "PNRC2"
}